{
  "term_id": "GO:0005886",
  "term_label": "plasma membrane",
  "gene_name": "Interleukin-18 receptor 1",
  "gene": "UniProtKB:Q13478",
  "gene_symbol": "IL18R1"
}